negative regulation of gibberellin biosynthetic process [GO:0010373] (biological process) Definition: Any process that stops, prevents, or reduces the frequency, rate or extent of the chemical reactions and pathways resulting in the formation of gibberellins. Also known as: negative regulation of gibberellic acid biosynthetic process Relationships: is a type of regulation of gibberellin biosynthetic process [GO:0010371]; is a type of negative regulation of isoprenoid metabolic process [GO:0045827]; is a type of GO:0051055; is_a GO:0062014; negatively regulates GO:0009686 Sources: GOC:tair_curators